{
  "gene": "UniProtKB:Q8NGX2",
  "gene_symbol": "OR2T35",
  "term_id": "GO:0050911",
  "gene_name": "Olfactory receptor 2T35",
  "term_label": "detection of chemical stimulus involved in sensory perception of smell"
}